Golgi stack lumen [GO:0034469] (cellular component) Relationships: is a type of GO:0005796; is part of Golgi stack [GO:0005795] Sources: GOC:mah Definition: The volume enclosed by any of the membranes of the thin, flattened cisternae that form the central portion of the Golgi complex.